{
  "gene_symbol": "MAP1A",
  "gene": "UniProtKB:P78559",
  "term_label": "synapse",
  "term_id": "GO:0045202",
  "gene_name": "Microtubule-associated protein 1A"
}